{
  "gene_symbol": "CDS2",
  "gene": "UniProtKB:O95674",
  "term_label": "endoplasmic reticulum membrane",
  "term_id": "GO:0005789",
  "gene_name": "Phosphatidate cytidylyltransferase 2"
}